{
  "gene_symbol": "SERTM1",
  "term_id": "UNKNOWN:0001",
  "term_label": "Unknown molecular function",
  "gene_name": "Serine-rich and transmembrane domain-containing protein 1",
  "gene": "UniProtKB:A2A2V5"
}